{
  "gene_name": "TOM1-like protein 2",
  "term_id": "GO:0016020",
  "gene": "UniProtKB:Q6ZVM7",
  "gene_symbol": "TOM1L2",
  "term_label": "membrane"
}